respiratory burst at fertilization [GO:0045729] (biological process) Definition: The phase of elevated metabolic activity, during which oxygen consumption increases, that occurs at fertilization. An enhanced uptake of oxygen leads to the production of hydrogen peroxide (H2O2), superoxide anions and hydroxyl radicals. Capacitation, a necessary prerequisite event to successful fertilization, can be induced by reactive oxygen species in vitro; hydrogen peroxide is used as an extracellular oxidant to cross-link the protective surface envelopes. Relationships: is a type of respiratory burst [GO:0045730]; BFO_0000050 single fertilization [GO:0007338] References: PMID:2537493, PMID:9013127 Sources: ISBN:0198506732 Also known as: metabolic burst at fertilization, oxidative burst at fertilization